response to thyroid hormone [GO:0097066] (biological process) Subtypes: cellular response to thyroid hormone stimulus [GO:0097067], response to thyroxine [GO:0097068] References: PMID:9916872 Sources: GOC:sjw Also known as: response to thyroid hormone stimulus Relationships: is a type of GO:0009725 Definition: A change in state or activity of a cell or an organism (in terms of movement, secretion, enzyme production, gene expression, etc.) as a result of a thyroid hormone stimulus.